{
  "term_id": "GO:0016567",
  "gene": "UniProtKB:Q9P0P0",
  "term_label": "protein ubiquitination",
  "gene_symbol": "RNF181",
  "gene_name": "E3 ubiquitin-protein ligase RNF181"
}